behavioral response to ether [GO:0048150] (biological process) Definition: Any process that results in a change in the behavior of an organism as a result of an ether stimulus. Sources: GOC:jid Also known as: behavioural response to ether Relationships: is a type of adult behavior [GO:0030534]; is part of response to ether [GO:0045472]